{
  "term_id": "GO:0005737",
  "term_label": "cytoplasm",
  "gene_name": "Coiled-coil domain-containing protein 88B",
  "gene": "UniProtKB:A6NC98",
  "gene_symbol": "CCDC88B"
}